{
  "gene_symbol": "SERINC3",
  "term_id": "UNKNOWN:0001",
  "gene_name": "Serine incorporator 3",
  "term_label": "Unknown molecular function",
  "gene": "UniProtKB:Q13530"
}